{
  "term_id": "GO:0042105",
  "gene": "UniProtKB:P04234",
  "gene_symbol": "CD3D",
  "term_label": "alpha-beta T cell receptor complex",
  "gene_name": "T-cell surface glycoprotein CD3 delta chain"
}